{
  "gene_symbol": "ZFP64",
  "term_id": "GO:0006355",
  "gene": "UniProtKB:Q9NTW7",
  "gene_name": "Zinc finger protein 64",
  "term_label": "regulation of DNA-templated transcription"
}